{
  "gene": "UniProtKB:P08582",
  "term_label": "extracellular space",
  "gene_name": "Melanotransferrin",
  "term_id": "GO:0005615",
  "gene_symbol": "MELTF"
}